{
  "term_label": "Unknown biological process",
  "gene": "UniProtKB:P46778",
  "gene_name": "Large ribosomal subunit protein eL21",
  "gene_symbol": "RPL21",
  "term_id": "UNKNOWN:0002"
}